{
  "gene_symbol": "ZNF311",
  "gene_name": "Zinc finger protein 311",
  "term_id": "GO:0005634",
  "gene": "UniProtKB:Q5JNZ3",
  "term_label": "nucleus"
}